{
  "gene_symbol": "S100A3",
  "term_label": "calcium-dependent protein binding",
  "gene_name": "Protein S100-A3",
  "term_id": "GO:0048306",
  "gene": "UniProtKB:P33764"
}